{
  "gene_name": "Growth arrest-specific protein 1",
  "gene": "UniProtKB:P54826",
  "term_id": "GO:0045930",
  "term_label": "negative regulation of mitotic cell cycle",
  "gene_symbol": "GAS1"
}